{
  "gene_symbol": "TWNK",
  "gene": "UniProtKB:Q96RR1",
  "term_id": "GO:0006264",
  "gene_name": "Twinkle mtDNA helicase",
  "term_label": "mitochondrial DNA replication"
}